{
  "gene": "UniProtKB:P10092",
  "gene_symbol": "CALCB",
  "term_label": "extracellular space",
  "term_id": "GO:0005615",
  "gene_name": "Calcitonin gene-related peptide 2"
}